{
  "gene_name": "Mitochondrial inner membrane protease ATP23 homolog",
  "gene": "UniProtKB:Q9Y6H3",
  "gene_symbol": "ATP23",
  "term_label": "Unknown cellular component",
  "term_id": "UNKNOWN:0003"
}